{
  "term_label": "microtubule",
  "gene_name": "Kinesin-like protein KIFC2",
  "term_id": "GO:0005874",
  "gene": "UniProtKB:Q96AC6",
  "gene_symbol": "KIFC2"
}